{
  "term_id": "GO:0030331",
  "gene": "UniProtKB:Q8N895",
  "gene_symbol": "ZNF366",
  "term_label": "nuclear estrogen receptor binding",
  "gene_name": "Zinc finger protein 366"
}